{
  "gene": "UniProtKB:Q9BV19",
  "term_label": "Unknown molecular function",
  "gene_symbol": "C1orf50",
  "gene_name": "Uncharacterized protein C1orf50",
  "term_id": "UNKNOWN:0001"
}